{
  "gene_symbol": "ANKRD35",
  "gene_name": "Ankyrin repeat domain-containing protein 35",
  "term_label": "Unknown molecular function",
  "term_id": "UNKNOWN:0001",
  "gene": "UniProtKB:Q8N283"
}